{
  "gene": "UniProtKB:Q9H6T0",
  "term_label": "nucleoplasm",
  "gene_name": "Epithelial splicing regulatory protein 2",
  "gene_symbol": "ESRP2",
  "term_id": "GO:0005654"
}